fumarylacetoacetase activity [GO:0004334] (molecular function) Definition: Catalysis of the reaction: 4-fumarylacetoacetate + H2O = acetoacetate + fumarate + H+. Also known as: 4-fumarylacetoacetate fumarylhydrolase activity, beta-diketonase activity, fumarylacetoacetate hydrolase activity Relationships: is_a hydrolase activity, acting on acid carbon-carbon bonds, in ketonic substances [GO:0016823] Sources: EC:3.7.1.2, RHEA:10244